endocardial progenitor cell migration to the midline involved in heart field formation [GO:0003262] (BP) Sources: GOC:mtg_heart Definition: The orderly movement of an endocardial progenitor cell toward the midline to form the heart field. Cardiac muscle progenitor cells are non-terminally differentiated, mesoderm-derived cells that are committed to differentiate into endocardial cells of the heart. Relationships: is a type of GO:0060975